{
  "gene_symbol": "DHFR",
  "term_id": "GO:0050661",
  "gene_name": "Dihydrofolate reductase",
  "term_label": "NADP binding",
  "gene": "UniProtKB:P00374"
}